otic placode formation [GO:0043049] (biological process) Relationships: is a type of ectodermal placode formation [GO:0060788]; is part of GO:0030916 Definition: The initial developmental process that will lead to the formation of the vertebrate inner ear. The otic placode forms as a thickening of the head ectoderm adjacent to the developing hindbrain. References: PMID:12668634 Sources: GOC:go_curators